negative regulation of male gonad development [GO:2000019] (biological process) Definition: Any process that stops, prevents, or reduces the frequency, rate or extent of male gonad development. Sources: GOC:obol, GOC:yaf Also known as: negative regulation of testicular development, negative regulation of testis development Relationships: is a type of GO:1905940; is a type of regulation of male gonad development [GO:2000018]; negatively regulates male gonad development [GO:0008584]